peroxisome proliferator activated receptor binding [GO:0042975] (molecular function) Relationships: is a type of signaling receptor binding [GO:0005102] Also known as: PPAR binding Definition: Binding to a peroxisome proliferator activated receptor, alpha, beta or gamma. References: PMID:12769781 Sources: GOC:jl